{
  "gene": "UniProtKB:Q96E39",
  "term_label": "mRNA binding",
  "gene_symbol": "RBMXL1",
  "term_id": "GO:0003729",
  "gene_name": "RNA binding motif protein, X-linked-like-1"
}